{
  "gene_name": "Large ribosomal subunit protein bL12m",
  "term_id": "GO:0003729",
  "gene": "UniProtKB:P52815",
  "gene_symbol": "MRPL12",
  "term_label": "mRNA binding"
}